{
  "term_label": "nucleus",
  "gene": "UniProtKB:Q9NRR4",
  "gene_symbol": "DROSHA",
  "term_id": "GO:0005634",
  "gene_name": "Ribonuclease 3"
}